{
  "term_id": "GO:0042981",
  "term_label": "regulation of apoptotic process",
  "gene_symbol": "NME2P1",
  "gene_name": "Putative nucleoside diphosphate kinase",
  "gene": "UniProtKB:O60361"
}